{
  "term_label": "steroid binding",
  "gene": "UniProtKB:P04278",
  "gene_name": "Sex hormone-binding globulin",
  "term_id": "GO:0005496",
  "gene_symbol": "SHBG"
}